{
  "gene_symbol": "HNRNPC",
  "term_label": "RNA binding",
  "gene": "UniProtKB:P07910",
  "term_id": "GO:0003723",
  "gene_name": "Heterogeneous nuclear ribonucleoproteins C1_C2"
}